{
  "gene_name": "Alanine and arginine-rich domain-containing protein",
  "term_label": "Unknown molecular function",
  "gene": "UniProtKB:Q4LEZ3",
  "gene_symbol": "AARD",
  "term_id": "UNKNOWN:0001"
}